{
  "gene_name": "E3 ubiquitin-protein ligase TRIM4",
  "term_id": "GO:0005737",
  "gene": "UniProtKB:Q9C037",
  "gene_symbol": "TRIM4",
  "term_label": "cytoplasm"
}